{
  "gene": "UniProtKB:O95750",
  "term_id": "GO:0008083",
  "term_label": "growth factor activity",
  "gene_name": "Fibroblast growth factor 19",
  "gene_symbol": "FGF19"
}